{
  "gene": "UniProtKB:Q86UP6",
  "gene_name": "CUB and zona pellucida-like domain-containing protein 1",
  "gene_symbol": "CUZD1",
  "term_label": "cell surface",
  "term_id": "GO:0009986"
}